follicular fluid formation in ovarian follicle antrum involved in scattered antral spaces stage [GO:0003005] (biological process) Also known as: follicular fluid formation in ovarian follicle antrum during scattered antral spaces stage Relationships: is a type of follicular fluid formation in ovarian follicle antrum [GO:0001548]; is part of GO:0048163 Sources: GOC:dph, GOC:isa_complete Definition: The menstrual cycle process in which one central cavity separating the oocyte/cumulus complex from mural granulosa and theca cells is formed as part of the scattered antral spaces stage of oogenesis.